{
  "gene": "UniProtKB:Q8TEQ8",
  "gene_name": "GPI ethanolamine phosphate transferase 3",
  "term_id": "GO:0051377",
  "gene_symbol": "PIGO",
  "term_label": "mannose-ethanolamine phosphotransferase activity"
}